dendrite guidance [GO:0070983] (biological process) Definition: The process in which the migration of a dendrite is directed to a specific target site in response to a combination of attractive and repulsive cues. Relationships: is a type of neuron projection guidance [GO:0097485]; is part of dendrite morphogenesis [GO:0048813] References: PMID:15046878 Sources: GOC:sart Also known as: dendritic guidance